{
  "term_id": "GO:1905515",
  "gene": "UniProtKB:O15078",
  "term_label": "non-motile cilium assembly",
  "gene_name": "Centrosomal protein of 290 kDa",
  "gene_symbol": "CEP290"
}